{
  "gene_name": "G antigen 12H",
  "gene_symbol": "GAGE12H",
  "term_id": "UNKNOWN:0001",
  "term_label": "Unknown molecular function",
  "gene": "UniProtKB:A6NDE8"
}